{
  "gene_name": "Olfactory receptor 1C1",
  "term_id": "GO:0004984",
  "term_label": "olfactory receptor activity",
  "gene": "UniProtKB:Q15619",
  "gene_symbol": "OR1C1"
}